deadenylation-independent decapping of nuclear-transcribed mRNA [GO:0031087] (biological process) Relationships: is a type of mRNA methylguanosine-cap decapping [GO:0110156]; is part of nuclear-transcribed mRNA catabolic process, deadenylation-independent decay [GO:0031086] References: PMID:15225542, PMID:15225544 Sources: GOC:krc Regulation: regulated by GO:1901834; positively regulated by positive regulation of deadenylation-independent decapping of nuclear-transcribed mRNA [GO:1901835] Also known as: deadenylylation-independent decapping, deadenylation-independent decapping of nuclear mRNA Definition: Cleavage of the 5'-cap of a nuclear-transcribed mRNA that is independent of poly(A) tail shortening. Subtypes: GO:0036450